{
  "term_id": "GO:0071007",
  "term_label": "U2-type catalytic step 2 spliceosome",
  "gene": "UniProtKB:Q9NW64",
  "gene_name": "Pre-mRNA-splicing factor RBM22",
  "gene_symbol": "RBM22"
}